{
  "gene_name": "Interferon regulatory factor 8",
  "gene_symbol": "IRF8",
  "term_id": "GO:0002376",
  "gene": "UniProtKB:Q02556",
  "term_label": "immune system process"
}